{
  "gene_name": "Prolyl 4-hydroxylase subunit alpha-2",
  "term_label": "Unknown biological process",
  "gene": "UniProtKB:O15460",
  "term_id": "UNKNOWN:0002",
  "gene_symbol": "P4HA2"
}